morphogenesis of larval imaginal disc epithelium [GO:0016335] (BP) Relationships: is a type of morphogenesis of an epithelium [GO:0002009]; is a type of post-embryonic animal morphogenesis [GO:0009886]; is part of instar larval development [GO:0002168]; is part of imaginal disc morphogenesis [GO:0007560] Definition: The process in which the anatomical structures of a larval imaginal disc epithelium are generated and organized. Sources: GOC:jl